DNA ligase activity [GO:0003909] (molecular function) Definition: Catalysis of the formation of a phosphodiester bond between the 3'-hydroxyl group at the end of one DNA chain and the 5'-phosphate group at the end of another. This reaction requires an energy source such as ATP or NAD+. Sources: ISBN:0716720094 Relationships: is a type of ligase activity, forming phosphoric ester bonds [GO:0016886]; is a type of catalytic activity, acting on DNA [GO:0140097] Subtypes: DNA ligase (ATP) activity [GO:0003910], GO:0003911